{
  "term_id": "GO:0007266",
  "gene_symbol": "EPS8",
  "gene": "UniProtKB:Q12929",
  "term_label": "Rho protein signal transduction",
  "gene_name": "Epidermal growth factor receptor kinase substrate 8"
}